{
  "term_id": "GO:0005886",
  "term_label": "plasma membrane",
  "gene_name": "E3 ubiquitin-protein ligase rififylin",
  "gene_symbol": "RFFL",
  "gene": "UniProtKB:Q8WZ73"
}